{
  "gene_name": "Mitochondrial dicarboxylate carrier",
  "term_id": "GO:0015116",
  "gene": "UniProtKB:Q9UBX3",
  "term_label": "sulfate transmembrane transporter activity",
  "gene_symbol": "SLC25A10"
}